{
  "gene": "UniProtKB:Q8WUH1",
  "gene_name": "Protein Churchill",
  "term_label": "Unknown cellular component",
  "gene_symbol": "CHURC1",
  "term_id": "UNKNOWN:0003"
}